periclinal cell division [GO:0090511] (BP) References: PMID:21391814 Sources: GOC:tair_curators Definition: A cell division process where the division plane is parallel to the surface of the organ. It creates a new cell layer or cell file. Relationships: is a type of GO:0051301